{
  "term_label": "protein complex involved in cell adhesion",
  "gene_name": "Junctional adhesion molecule C",
  "gene_symbol": "JAM3",
  "term_id": "GO:0098636",
  "gene": "UniProtKB:Q9BX67"
}